regulation of nonadec-1-ene biosynthetic process [GO:1900935] (biological process) Sources: GOC:TermGenie, GOC:mengo_curators Also known as: regulation of nonadec-1-ene anabolism, regulation of nonadec-1-ene biosynthesis, regulation of nonadec-1-ene formation, regulation of nonadec-1-ene synthesis Relationships: is a type of regulation of olefin biosynthetic process [GO:1900911]; regulates nonadec-1-ene biosynthetic process [GO:1900877] Subtypes: GO:1900936, positive regulation of nonadec-1-ene biosynthetic process [GO:1900937] Definition: Any process that modulates the frequency, rate or extent of nonadec-1-ene biosynthetic process.